stomatal lineage progression [GO:0010440] (biological process) Relationships: is a type of cellular developmental process [GO:0048869]; is part of stomatal complex development [GO:0010374] Definition: The process in which an unspecialized epidermal cell progresses through a series of divisions that culminate in the production of a stomatal complex. Sources: GOC:expert_db, GOC:tb